ventral spinal cord interneuron differentiation [GO:0021514] (biological process) Relationships: is a type of GO:0021515; is a type of central nervous system neuron differentiation [GO:0021953]; is part of ventral spinal cord development [GO:0021517] Definition: The process in which neuroepithelial cells in the neural tube acquire specialized structural and/or functional features of ventral spinal cord interneurons. Ventral spinal cord interneurons are cells located in the ventral portion of the spinal cord that transmit signals between sensory and motor neurons and are required for reflexive responses. Differentiation includes the processes involved in commitment of a cell to a specific fate. References: PMID:11262869 Sources: GOC:cls, GOC:dgh, GOC:dph, GOC:jid, GO_REF:0000021